{
  "gene_symbol": "MOCS1",
  "term_label": "Mo-molybdopterin cofactor biosynthetic process",
  "term_id": "GO:0006777",
  "gene_name": "Molybdenum cofactor biosynthesis protein 1",
  "gene": "UniProtKB:Q9NZB8"
}